{
  "term_id": "UNKNOWN:0002",
  "term_label": "Unknown biological process",
  "gene_symbol": "MEA1",
  "gene": "UniProtKB:Q16626",
  "gene_name": "Male-enhanced antigen 1"
}